{
  "term_id": "GO:0005634",
  "term_label": "nucleus",
  "gene": "UniProtKB:Q13164",
  "gene_name": "Mitogen-activated protein kinase 7",
  "gene_symbol": "MAPK7"
}